{
  "term_label": "GPI anchor biosynthetic process",
  "gene_symbol": "PIGP",
  "gene_name": "Phosphatidylinositol N-acetylglucosaminyltransferase subunit P",
  "gene": "UniProtKB:P57054",
  "term_id": "GO:0006506"
}